negative regulation of mitotic cytokinetic process [GO:1903437] (biological process) Relationships: is a type of negative regulation of mitotic cytokinesis [GO:1902413]; is_a GO:1903436; negatively regulates mitotic cytokinetic process [GO:1902410] Subtypes: negative regulation of mitotic division septum assembly [GO:0140280], negative regulation of mitotic actomyosin contractile ring contraction [GO:1903472], negative regulation of mitotic actomyosin contractile ring assembly [GO:1903500] Definition: Any process that stops, prevents or reduces the frequency, rate or extent of mitotic cytokinetic process. Also known as: down regulation of mitotic cytokinetic process, down-regulation of mitotic cytokinetic process, downregulation of mitotic cytokinetic process, inhibition of mitotic cytokinetic process Sources: GOC:TermGenie, GOC:vw, GO_REF:0000058